{
  "gene_name": "Coiled-coil domain-containing protein 89",
  "term_id": "UNKNOWN:0002",
  "gene_symbol": "CCDC89",
  "gene": "UniProtKB:Q8N998",
  "term_label": "Unknown biological process"
}